mitochondrial promoter sequence-specific DNA binding [GO:0001018] (molecular function) Also known as: HSP coding strand binding, HSP non-coding strand binding, HSPas binding, HSPs binding, LSP coding strand binding, LSP non-coding strand binding, LSPas binding, LSPs binding, mitochondrial heavy strand promoter anti-sense binding, mitochondrial heavy strand promoter sense binding, mitochondrial light strand promoter anti-sense binding, mitochondrial light strand promoter sense binding, mitochondrial RNA polymerase core promoter proximal region sequence-specific DNA binding, mitochondrial RNA polymerase core promoter sequence-specific DNA binding, mitochondrial RNA polymerase regulatory region DNA binding, mitochondrial RNA polymerase regulatory region sequence-specific DNA binding, mitochondrial proximal promoter sequence-specific DNA binding Definition: Binding to a DNA region that controls the transcription of the mitochondrial DNA. References: PMID:20056105 Sources: GOC:txnOH, GOC:vw Relationships: is a type of transcription cis-regulatory region binding [GO:0000976]